proplastid stroma [GO:0009571] (cellular component) Relationships: is a type of plastid stroma [GO:0009532]; is part of proplastid [GO:0009537] Sources: GOC:jl Definition: The space enclosed by the double membrane of a proplastid.